antigen transcytosis by M cells in mucosal-associated lymphoid tissue [GO:0002412] (biological process) References: PMID:12843411 Sources: GOC:jal, ISBN:0781735149 Relationships: is a type of transcytosis [GO:0045056]; is part of GO:0002406 Also known as: antigen transcytosis by M cells in MALT, antigen transport by M cells in MALT, antigen transport by M cells in mucosal-associated lymphoid tissue Definition: The process of antigen transcytosis carried out by M cells in the mucosal-associated lymphoid tissue (MALT). Transcytosis is the process of the directed movement of endocytosed material through the cell and its exocytosis from the plasma membrane at the opposite side. M cells are specialized epithelia cells with a microfold structure that are adept at moving antigens from the gut lumen to antigen presenting cells in the MALT.